sex comb development [GO:0045498] (biological process) Definition: The process whose specific outcome is the progression of the sex comb over time, from its formation to the mature structure. The sex combs are the male specific chaetae located on the prothoracic tarsal segment of the prothoracic leg. Sources: http://fly.ebi.ac.uk Relationships: is a type of GO:0007423